{
  "gene_symbol": "TRAV30",
  "term_label": "Unknown molecular function",
  "gene": "UniProtKB:A0A087WSZ9",
  "gene_name": "T cell receptor alpha variable 30",
  "term_id": "UNKNOWN:0001"
}